{
  "term_id": "UNKNOWN:0002",
  "term_label": "Unknown biological process",
  "gene_symbol": "FAM74A1",
  "gene": "UniProtKB:Q5RGS3",
  "gene_name": "Protein FAM74A1"
}